uroporphyrinogen III metabolic process [GO:0046502] (biological process) Definition: The chemical reactions and pathways involving uroporphyrinogen III, a precursor for synthesis of vitamin B12, chlorophyll, and heme in organisms that produce these compounds. Also known as: uroporphyrinogen III metabolism Relationships: is a type of porphyrin-containing compound metabolic process [GO:0006778]; is a type of carboxylic acid metabolic process [GO:0019752] Subtypes: uroporphyrinogen III biosynthetic process [GO:0006780] Sources: GOC:ai